positive regulation of peptide hormone secretion [GO:0090277] (biological process) Relationships: is_a positive regulation of peptide secretion [GO:0002793]; is a type of GO:0046887; is a type of regulation of peptide hormone secretion [GO:0090276]; positively regulates peptide hormone secretion [GO:0030072] Sources: GOC:tb Subtypes: GO:0032024, positive regulation of corticotropin secretion [GO:0051461], positive regulation of corticotropin-releasing hormone secretion [GO:0051466], positive regulation of growth hormone secretion [GO:0060124], positive regulation of glucagon secretion [GO:0070094], positive regulation of somatostatin secretion [GO:0090274], positive regulation of prolactin secretion [GO:1902722], GO:1904364, positive regulation of substance P secretion [GO:1904460], positive regulation of thyroid-stimulating hormone secretion [GO:2000614] Definition: Any process that increases the rate, frequency, or extent of the regulated release of a peptide hormone from secretory granules.